{
  "gene": "UniProtKB:Q9H9L3",
  "term_id": "GO:0004527",
  "gene_name": "Interferon-stimulated 20 kDa exonuclease-like 2",
  "term_label": "exonuclease activity",
  "gene_symbol": "ISG20L2"
}